{
  "term_label": "B cell activation involved in immune response",
  "term_id": "GO:0002312",
  "gene": "UniProtKB:P05000",
  "gene_symbol": "IFNW1",
  "gene_name": "Interferon omega-1"
}